{
  "gene_symbol": "POLR2E",
  "gene_name": "DNA-directed RNA polymerases I, II, and III subunit RPABC1",
  "term_id": "GO:0003899",
  "term_label": "DNA-directed RNA polymerase activity",
  "gene": "UniProtKB:P19388"
}